{
  "term_label": "lipid transport",
  "gene_symbol": "ABCA8",
  "gene_name": "ABC-type organic anion transporter ABCA8",
  "gene": "UniProtKB:O94911",
  "term_id": "GO:0006869"
}